regulation of sulfite transmembrane transport [GO:1900071] (biological process) Relationships: is a type of regulation of transmembrane transport [GO:0034762]; regulates GO:0000316 Definition: Any process that modulates the frequency, rate or extent of sulfite transmembrane transport. References: PMID:10234785, PMID:10870099 Sources: GOC:TermGenie Also known as: regulation of sulfite transport, regulation of sulphite transport Subtypes: GO:1900072